{
  "term_id": "GO:0005730",
  "gene": "UniProtKB:Q9NX58",
  "term_label": "nucleolus",
  "gene_name": "Cell growth-regulating nucleolar protein",
  "gene_symbol": "LYAR"
}